{
  "gene": "UniProtKB:Q969P6",
  "gene_symbol": "TOP1MT",
  "gene_name": "DNA topoisomerase I, mitochondrial",
  "term_id": "GO:0006265",
  "term_label": "DNA topological change"
}